{
  "gene_symbol": "RAB6D",
  "gene_name": "Ras-related protein Rab-6D",
  "term_label": "intracellular protein transport",
  "gene": "UniProtKB:Q53S08",
  "term_id": "GO:0006886"
}